regulation of T cell mediated cytotoxicity [GO:0001914] (biological process) Definition: Any process that modulates the frequency, rate, or extent of T cell mediated cytotoxicity. Sources: GOC:add, ISBN:0781735149 Relationships: is a type of GO:0001910; is a type of regulation of T cell mediated immunity [GO:0002709]; regulates T cell mediated cytotoxicity [GO:0001913] Also known as: regulation of T cell mediated apoptosis, regulation of T cell mediated cell death, regulation of T cell mediated cell killing, regulation of T lymphocyte mediated cytotoxicity, regulation of T-cell mediated apoptosis, regulation of T-cell mediated cell death, regulation of T-cell mediated cell killing, regulation of T-cell mediated cytotoxicity, regulation of T-lymphocyte mediated cytotoxicity, regulation of T cell mediated cytolysis, regulation of T-cell mediated cytolysis Subtypes: negative regulation of T cell mediated cytotoxicity [GO:0001915], positive regulation of T cell mediated cytotoxicity [GO:0001916], regulation of T cell mediated cytotoxicity directed against tumor cell target [GO:0002852], regulation of cytotoxic T cell degranulation [GO:0043317]